{
  "term_id": "GO:0006338",
  "term_label": "chromatin remodeling",
  "gene_name": "Transcriptional repressor p66-beta",
  "gene_symbol": "GATAD2B",
  "gene": "UniProtKB:Q8WXI9"
}